negative regulation of host-seeking behavior [GO:0032539] (biological process) Relationships: is a type of GO:0032538; is a type of negative regulation of behavior [GO:0048521]; negatively regulates host-seeking behavior [GO:0032537] Also known as: down regulation of host-seeking behavior, down-regulation of host-seeking behavior, downregulation of host-seeking behavior, negative regulation of host-seeking behaviour, inhibition of host-seeking behavior Definition: Any process that stops, prevents, or reduces the frequency, rate or extent of any behavior associated with finding a host organism. Sources: GOC:mah